{
  "gene_symbol": "CYP2B6",
  "term_id": "GO:0008392",
  "gene": "UniProtKB:P20813",
  "gene_name": "Cytochrome P450 2B6",
  "term_label": "arachidonate epoxygenase activity"
}